{
  "gene": "UniProtKB:Q86XE0",
  "term_id": "GO:0042147",
  "gene_name": "Sorting nexin-32",
  "term_label": "retrograde transport, endosome to Golgi",
  "gene_symbol": "SNX32"
}